{
  "term_id": "GO:0016165",
  "gene": "UniProtKB:P18054",
  "term_label": "linoleate 13S-lipoxygenase activity",
  "gene_symbol": "ALOX12",
  "gene_name": "Polyunsaturated fatty acid lipoxygenase ALOX12"
}